{
  "gene_name": "Ribosomal protein S6 kinase-related protein",
  "term_label": "Unknown cellular component",
  "term_id": "UNKNOWN:0003",
  "gene_symbol": "RSKR",
  "gene": "UniProtKB:Q96LW2"
}